neural plate pattern specification [GO:0060896] (biological process) Sources: GOC:dph, GOC:sdb_2009, GOC:tb Definition: The developmental process that results in the creation of defined areas or spaces within the neural plate to which cells respond and eventually are instructed to differentiate. Subtypes: neural plate regionalization [GO:0060897] Relationships: is a type of pattern specification process [GO:0007389]